immune complex clearance [GO:0002434] (biological process) Relationships: is_a immune effector process [GO:0002252] Subtypes: immune complex clearance by erythrocytes [GO:0002435], immune complex clearance by monocytes and macrophages [GO:0002436] Sources: GOC:add, GO_REF:0000022, ISBN:068340007X Definition: A process directed at removing immune complexes from the body. Immune complexes are clusters of antibodies bound to antigen, to which complement may also be fixed, and which may precipitate or remain in solution.